prespliceosome [GO:0071010] (cellular component) Relationships: is a type of spliceosomal complex [GO:0005681] Definition: A spliceosomal complex that is formed by association of the 5' splice site and the branch point sequence with specific snRNPs. The prespliceosome includes many proteins in addition to those found in the bound snRNPs. Commitment to a given pair of 5' and 3' splice sites occurs at the time of prespliceosome formation. Prespliceosome complexes are not active for splicing, but are instead an early step in the assembly of a spliceosomal complex. References: PMID:17332742, PMID:19239890 Sources: GOC:ab, GOC:krc, GOC:mah Also known as: prespliceosomal complex, mammalian spliceosomal complex A, yeast spliceosomal complex B Subtypes: U2-type prespliceosome [GO:0071004], GO:0071015